{
  "gene_name": "E3 SUMO-protein ligase PIAS1",
  "gene": "UniProtKB:O75925",
  "term_id": "GO:0006357",
  "gene_symbol": "PIAS1",
  "term_label": "regulation of transcription by RNA polymerase II"
}